meiotic cell cycle process [GO:1903046] (biological process) Relationships: is a type of GO:0022402; is a type of reproductive process [GO:0022414]; is part of meiotic cell cycle [GO:0051321] Sources: GOC:TermGenie, GOC:mtg_cell_cycle, GO_REF:0000060 Subtypes: meiotic spindle organization [GO:0000212], meiotic DNA double-strand break processing [GO:0000706], meiotic joint molecule formation [GO:0000709], GO:0006279, reciprocal meiotic recombination [GO:0007131], meiotic chromosome movement towards spindle pole [GO:0016344], ascospore formation [GO:0030437], ascospore wall assembly [GO:0030476], dynein-driven meiotic oscillatory nuclear movement [GO:0030989], linear element assembly [GO:0030999], ascospore-type prospore assembly [GO:0031321], ascospore-type prospore-specific spindle pole body remodeling [GO:0031322], horsetail-astral microtubule organization [GO:0032118], ascospore-type prospore membrane formation [GO:0032120], meiotic attachment of telomeric heterochromatin to spindle pole body [GO:0032121], meiotic cytokinesis [GO:0033206], meiotic cell cycle checkpoint signaling [GO:0033313], sexual spore wall assembly [GO:0034294], ascospore wall beta-glucan metabolic process [GO:0034408], meiotic cell cycle phase transition [GO:0044771], meiotic chromosome segregation [GO:0045132], plant-type sporogenesis [GO:0048236], GO:0051026, GO:0051078, meiotic spindle elongation [GO:0051232], meiotic spindle midzone assembly [GO:0051257], establishment of meiotic spindle localization [GO:0051295], GO:0051307, meiotic metaphase chromosome alignment [GO:0051311], GO:0051316, meiotic nuclear membrane reassembly [GO:0051333], meiotic sister chromatid arm separation [GO:0051755], GO:0051756, lateral element assembly [GO:0051878], meiosis I cell cycle process [GO:0061982], GO:0061983, LinE complex assembly [GO:0062120], GO:0070192, meiotic attachment of telomere to nuclear envelope [GO:0070197], spore membrane bending pathway [GO:0070583], ascospore wall biogenesis [GO:0070591], ascospore release from ascus [GO:0071998], response to meiotic recombination checkpoint signaling [GO:0072461], GO:0140013, initial meiotic spindle pole body separation [GO:0140456], meiotic DNA replication initiation [GO:1902974], premeiotic DNA replication preinitiation complex assembly [GO:1902976], premeiotic DNA replication termination [GO:1902978], GO:1902982, pre-replicative complex assembly involved in premeiotic DNA replication [GO:1902984], meiotic cell cycle process involved in oocyte maturation [GO:1903537], GO:1903563, GO:1904967, GO:1990395, meiotic centromeric cohesion protection in anaphase I [GO:1990813], double-strand break repair involved in meiotic recombination [GO:1990918] Definition: A process that is part of the meiotic cell cycle.